{
  "term_label": "Unknown cellular component",
  "gene_name": "Transmembrane protein 116",
  "gene_symbol": "TMEM116",
  "gene": "UniProtKB:Q8NCL8",
  "term_id": "UNKNOWN:0003"
}